acrosomal membrane [GO:0002080] (cellular component) Relationships: is a type of secretory granule membrane [GO:0030667]; is part of acrosomal vesicle [GO:0001669] Sources: GOC:dph Definition: The membrane that surrounds the acrosomal lumen. The acrosome is a special type of lysosome in the head of a spermatozoon that contains acid hydrolases and is concerned with the breakdown of the outer membrane of the ovum during fertilization.